trans-translation [GO:0070929] (biological process) Definition: A translational elongation process in which transfer of a translating ribosome from one mRNA to another RNA template takes place. Trans-translation occurs during tmRNA release of stalled ribosomes. Sources: GOC:jh2, GOC:mah Relationships: is a type of GO:0006414